arginine catabolic process to alanine via ornithine [GO:0010122] (biological process) Relationships: is a type of alanine metabolic process [GO:0006522]; is_a arginine metabolic process [GO:0006525]; is a type of alpha-amino acid catabolic process [GO:1901606] Definition: The chemical reactions and pathways resulting in the breakdown of arginine into other compounds, including alanine, via ornithine. Sources: GOC:pz Also known as: arginine breakdown to alanine via ornithine, arginine degradation to alanine via ornithine